16S rRNA (adenine(1518)-N(6)/adenine(1519)-N(6))-dimethyltransferase activity [GO:0052908] (molecular function) Definition: Catalysis of the reaction: 4 S-adenosyl-L-methionine + adenine(1518)/adenine(1519) in 16S rRNA = 4 S-adenosyl-L-homocysteine + N(6)-dimethyladenine(1518)/N(6)-dimethyladenine(1519) in 16S rRNA. Sources: RHEA:19609 Also known as: S-adenosylmethionine-6-N',N'-adenosyl (rRNA) dimethyltransferase activity Relationships: is_a rRNA (adenine-N6,N6-)-dimethyltransferase activity [GO:0000179]